tolerance induction to tumor cell [GO:0002413] (biological process) Definition: A process of tolerance induction which leads to immunological tolerance of a tumor. Sources: GOC:add Relationships: is a type of GO:0002418; is a type of peripheral tolerance induction [GO:0002465] Subtypes: T cell tolerance induction to tumor cell [GO:0002411] Regulation: regulated by regulation of tolerance induction to tumor cell [GO:0002843]; negatively regulated by GO:0002844; positively regulated by positive regulation of tolerance induction to tumor cell [GO:0002845]